intracellular auxin homeostasis [GO:0140964] (BP) Definition: A homeostatic process involved in the maintenance of a steady state level of auxin within a cell. Relationships: is a type of intracellular chemical homeostasis [GO:0055082] References: PMID:19506555, PMID:22314799 Also known as: auxin homeostasis, cellular auxin homeostasis